{
  "gene_symbol": "KRR1",
  "gene": "UniProtKB:Q13601",
  "gene_name": "KRR1 small subunit processome component homolog",
  "term_label": "Unknown biological process",
  "term_id": "UNKNOWN:0002"
}